karyogamy involved in conjugation with mutual genetic exchange [GO:0000744] (biological process) Sources: GOC:mah, GOC:pg Definition: During sexual reproduction, the creation of a single nucleus from two nuclei as a result of fusing the nuclear envelopes that surround each nuclei. This takes place following the mutual exchange of one of the two nuclei produced by the mitosis that follows the second meiotic nuclear division. This occurs in ciliated protozoans such as Tetrahymena. Relationships: is a type of karyogamy [GO:0000741]; is part of conjugation with mutual genetic exchange [GO:0000748] Also known as: karyogamy involved in conjugation without cellular fusion